positive regulation of meiotic cell cycle [GO:0051446] (biological process) Relationships: is a type of positive regulation of cell cycle [GO:0045787]; is a type of regulation of meiotic cell cycle [GO:0051445]; is a type of positive regulation of reproductive process [GO:2000243]; positively regulates meiotic cell cycle [GO:0051321] Definition: Any process that activates or increases the frequency, rate or extent of progression through the meiotic cell cycle. Subtypes: GO:0043941, positive regulation of meiotic nuclear division [GO:0045836], GO:0051728, GO:0140648, positive regulation of meiotic cell cycle phase transition [GO:1901995], positive regulation of meiotic cell cycle process involved in oocyte maturation [GO:1904146] Also known as: positive regulation of meiotic cell cycle progression, positive regulation of progression through meiotic cell cycle, up regulation of progression through meiotic cell cycle, up-regulation of progression through meiotic cell cycle, upregulation of progression through meiotic cell cycle, activation of progression through meiotic cell cycle, stimulation of progression through meiotic cell cycle Sources: GOC:ai, GOC:dph, GOC:tb